{
  "gene": "UniProtKB:Q9UJX3",
  "term_id": "GO:0005680",
  "gene_symbol": "ANAPC7",
  "term_label": "anaphase-promoting complex",
  "gene_name": "Anaphase-promoting complex subunit 7"
}